mandelate biosynthetic process [GO:0046236] (biological process) Definition: The chemical reactions and pathways resulting in the formation of mandelate, the anion of mandelic acid. Mandelic acid (alpha-hydroxybenzeneacetic acid) is an 8-carbon alpha-hydroxy acid (AHA) that is used in organic chemistry and as a urinary antiseptic. Sources: GOC:ai Relationships: is a type of mandelate metabolic process [GO:0018924]; is a type of monocarboxylic acid biosynthetic process [GO:0072330] Also known as: mandelate anabolism, mandelate biosynthesis, mandelate formation, mandelate synthesis